tetrose metabolic process [GO:0033347] (biological process) Subtypes: tetrose biosynthetic process [GO:0033348] Relationships: is a type of monosaccharide metabolic process [GO:0005996] Definition: The chemical reactions and pathways involving a tetrose, any monosaccharide with a chain of four carbon atoms in the molecule. Sources: GOC:mah Also known as: tetrose metabolism